{
  "gene_name": "DNA-directed RNA polymerases I, II, and III subunit RPABC2",
  "gene": "UniProtKB:P61218",
  "term_id": "GO:0005736",
  "term_label": "RNA polymerase I complex",
  "gene_symbol": "POLR2F"
}